{
  "gene_name": "Protein transport protein Sec61 subunit beta",
  "term_label": "Sec61 translocon complex",
  "gene_symbol": "SEC61B",
  "term_id": "GO:0005784",
  "gene": "UniProtKB:P60468"
}